{
  "gene_name": "Ubiquitin carboxyl-terminal hydrolase 17-like protein 15",
  "gene": "UniProtKB:C9J2P7",
  "gene_symbol": "USP17L15",
  "term_label": "nucleus",
  "term_id": "GO:0005634"
}